{
  "term_id": "GO:0048205",
  "term_label": "COPI coating of Golgi vesicle",
  "gene": "UniProtKB:Q8N6H7",
  "gene_symbol": "ARFGAP2",
  "gene_name": "ADP-ribosylation factor GTPase-activating protein 2"
}